mitochondrial RNA surveillance [GO:2000827] (biological process) Definition: The set of processes involved in identifying and degrading defective or aberrant RNAs that takes place in the mitochondrion. References: PMID:19864255 Also known as: RNA quality control in mitochondria, RNA quality control in mitochondrion, RNA surveillance in mitochondria, aberrant RNA catabolic process in mitochondria, aberrant RNA catabolic process in mitochondrion Relationships: is a type of mitochondrial RNA catabolic process [GO:0000957]; is a type of cytoplasmic RNA surveillance [GO:0071026] Subtypes: mitochondrial ncRNA surveillance [GO:0035945], mitochondrial mRNA surveillance [GO:0035946]